{
  "term_label": "epoxide metabolic process",
  "term_id": "GO:0097176",
  "gene": "UniProtKB:P07099",
  "gene_name": "Epoxide hydrolase 1",
  "gene_symbol": "EPHX1"
}